{
  "gene_name": "Glutaminyl-peptide cyclotransferase-like protein",
  "gene": "UniProtKB:Q9NXS2",
  "term_id": "UNKNOWN:0002",
  "gene_symbol": "QPCTL",
  "term_label": "Unknown biological process"
}